histone H3K36 demethylase activity [GO:0051864] (molecular function) Note: Comment: Note that the residue position corresponds to the canonical human H3 histone (UniProtKB:P84243); this residue is conserved across all eukaryotes. Residue 1 is the first residue following removal of the initiating Methionine (Met). Note that each histone is encoded by multiple genes, and sequences may vary across different genes within an organism. Also known as: [histone-H3]-lysine-36 demethylase activity, histone H3-K36 demethylase activity, histone H3-lysine-36 demethylase activity, histone H3-methyl-lysine-36 demethylase activity, histone demethylase activity (H3-K36 specific), histone-lysine (H3-K36) demethylase activity, histone-lysine demethylase activity (H3-K36 specific), histone-lysine(H3-K36) demethylase activity References: PMID:16362057 Definition: Catalysis of the removal of a methyl group from a modified lysine residue at position 36 of the histone H3 protein. This is a dioxygenase reaction that is dependent on Fe(II) and 2-oxoglutarate. Subtypes: GO:0140680, histone H3K36me2/H3K36me3 demethylase activity [GO:0140681] Relationships: is_a 2-oxoglutarate-dependent dioxygenase activity [GO:0016706]; is a type of GO:0141052